translocation of peptides or proteins into host cell cytoplasm [GO:0044053] (biological process) Definition: The directed movement of peptides or proteins produced by a symbiont organism to a location within the host cell cytoplasm. Sources: MITRE:tk Also known as: translocation of symbiont peptides or proteins into host cell cytoplasm, transport of peptides or proteins into host cell cytoplasm Relationships: is a type of translocation of peptides or proteins into host [GO:0042000]